{
  "term_id": "GO:0000978",
  "term_label": "RNA polymerase II cis-regulatory region sequence-specific DNA binding",
  "gene_name": "Max-binding protein MNT",
  "gene_symbol": "MNT",
  "gene": "UniProtKB:Q99583"
}